{
  "gene": "UniProtKB:Q8IZU0",
  "term_id": "GO:0000795",
  "term_label": "synaptonemal complex",
  "gene_name": "Protein FAM9B",
  "gene_symbol": "FAM9B"
}